{
  "gene": "UniProtKB:O15033",
  "gene_symbol": "AREL1",
  "gene_name": "Apoptosis-resistant E3 ubiquitin protein ligase 1",
  "term_id": "GO:0005737",
  "term_label": "cytoplasm"
}